{
  "gene_symbol": "ZNF362",
  "gene": "UniProtKB:Q5T0B9",
  "gene_name": "Zinc finger protein 362",
  "term_label": "RNA polymerase II cis-regulatory region sequence-specific DNA binding",
  "term_id": "GO:0000978"
}